{
  "gene_symbol": "CUTA",
  "term_id": "GO:0005507",
  "gene": "UniProtKB:O60888",
  "gene_name": "Protein CutA",
  "term_label": "copper ion binding"
}